{
  "term_label": "Unknown molecular function",
  "gene": "UniProtKB:O15394",
  "gene_name": "Neural cell adhesion molecule 2",
  "term_id": "UNKNOWN:0001",
  "gene_symbol": "NCAM2"
}